{
  "term_id": "GO:0006511",
  "gene_name": "F-box only protein 10",
  "term_label": "ubiquitin-dependent protein catabolic process",
  "gene_symbol": "FBXO10",
  "gene": "UniProtKB:Q9UK96"
}